malate synthase activity [GO:0004474] (molecular function) Definition: Catalysis of the reaction: acetyl-CoA + glyoxylate + H2O = (S)-malate + CoA + H+. Sources: RHEA:18181 Also known as: L-malate glyoxylate-lyase (CoA-acetylating) activity, acetyl-CoA:glyoxylate C-acetyltransferase (thioester-hydrolysing, carboxymethyl-forming), glyoxylate transacetase activity, glyoxylate transacetylase activity, glyoxylic transacetase activity, malate condensing enzyme activity, malate synthetase activity, malic synthetase activity, malic-condensing enzyme activity Relationships: is a type of acyltransferase activity, acyl groups converted into alkyl on transfer [GO:0046912]